inositol 1-methyltransferase activity [GO:0030741] (molecular function) Definition: Catalysis of the reaction: S-adenosyl-L-methionine(1+) + myo-inositol = 1D-1-O-methyl-myo-inositol + S-adenosyl-L-homocysteine + H+. Sources: EC:2.1.1.40, RHEA:17565 Relationships: is_a GO:0008757 Also known as: S-adenosyl-L-methionine:1D-myo-inositol 1-O-methyltransferase activity, S-adenosyl-L-methionine:myo-inositol 3-O-methyltransferase activity, S-adenosylmethionine:myo-inositol 3-methyltransferase activity, inositol 3-O-methyltransferase (name based on 1L-numbering system and not 1D-numbering), inositol 3-O-methyltransferase activity, inositol D-1-methyltransferase activity, myo-inositol 3-O-methyltransferase activity